{
  "term_label": "ATP binding",
  "gene": "UniProtKB:Q12931",
  "gene_name": "Heat shock protein 75 kDa, mitochondrial",
  "term_id": "GO:0005524",
  "gene_symbol": "TRAP1"
}